N-terminal protein amino acid modification [GO:0031365] (biological process) Subtypes: N-terminal protein amino acid acetylation [GO:0006474], N-terminal protein amino acid methylation [GO:0006480], N-terminal protein lipidation [GO:0006498], N-terminal protein formylation [GO:0018004], N-terminal protein amino acid deamination [GO:0031363], N-terminal protein amino acid carboxylation [GO:0050989], N-terminal protein amino acid carbamoylation [GO:0050990] Also known as: peptide or protein amino-terminal blocking, peptide/protein amino-terminal blocking Definition: The alteration of the N-terminal amino acid residue in a protein. Relationships: is a type of protein modification process [GO:0036211] Sources: GOC:mah